7-methylguanosine metabolic process [GO:0008618] (biological process) Definition: The chemical reactions and pathways involving 7-methylguanosine, a modified nucleoside that forms a cap at the 5'-terminus of eukaryotic mRNA. Relationships: is a type of GO:0046128 Sources: ISBN:0198506732 Also known as: 7-methylguanosine metabolism Subtypes: 7-methylguanosine biosynthetic process [GO:0046118], 7-methylguanosine catabolic process [GO:0046119]